{
  "gene_name": "TERF1-interacting nuclear factor 2",
  "gene": "UniProtKB:Q9BSI4",
  "gene_symbol": "TINF2",
  "term_id": "GO:0042162",
  "term_label": "telomeric DNA binding"
}